{
  "gene": "UniProtKB:Q05329",
  "gene_name": "Glutamate decarboxylase 2",
  "term_label": "cytoplasm",
  "term_id": "GO:0005737",
  "gene_symbol": "GAD2"
}